glucose transporter complex [GO:1990350] (cellular component) Definition: A protein complex facilitating glucose transport into, out of or within a cell, or between cells. References: PMID:15449578 Sources: GOC:bhm Note: An example of this is GTR1 in human (UniProt symbol P11166) in PMID:15449578 (inferred from direct assay). Relationships: is a type of transporter complex [GO:1990351]